{
  "gene_symbol": "ZNF845",
  "term_id": "GO:0005634",
  "term_label": "nucleus",
  "gene": "UniProtKB:Q96IR2",
  "gene_name": "Zinc finger protein 845"
}